{
  "term_label": "nucleolus",
  "gene_name": "Probable ATP-dependent RNA helicase DDX56",
  "gene_symbol": "DDX56",
  "gene": "UniProtKB:Q9NY93",
  "term_id": "GO:0005730"
}